mechanosensory lateral line system development [GO:0048881] (biological process) Definition: The process whose specific outcome is the progression of the mechanosensory lateral line system over time, from its formation to the mature structure. The mechanosensory lateral line system consists of small sensory patches (neuromasts) located superficially on the skin or just under the skin in fluid-filled canals on the head and body of all fishes and most amphibians. The neuromasts are innervated by several lateral line nerves, which project primarily to the hindbrain. The mechanosensory lateral line system is stimulated by local water displacements and vibrations, and detects propulsion of the fish through the water, as well as facilitating shoaling, prey capture, and predator and obstacle avoidance. Sources: ISBN:0125296509 Also known as: LL system development Relationships: is a type of GO:0048925